{
  "gene_name": "All trans-polyprenyl-diphosphate synthase PDSS1",
  "term_label": "ubiquinone biosynthetic process",
  "term_id": "GO:0006744",
  "gene_symbol": "PDSS1",
  "gene": "UniProtKB:Q5T2R2"
}